{
  "gene_name": "T cell receptor alpha variable 19",
  "gene": "UniProtKB:A0A0A6YYK7",
  "term_id": "GO:0006955",
  "gene_symbol": "TRAV19",
  "term_label": "immune response"
}